{
  "gene": "UniProtKB:P61457",
  "gene_name": "Pterin-4-alpha-carbinolamine dehydratase",
  "term_label": "Unknown cellular component",
  "gene_symbol": "PCBD1",
  "term_id": "UNKNOWN:0003"
}